{
  "term_label": "Unknown cellular component",
  "gene_symbol": "NUTM2F",
  "gene_name": "NUT family member 2F",
  "term_id": "UNKNOWN:0003",
  "gene": "UniProtKB:A1L443"
}